{
  "term_label": "CORVET complex",
  "gene_name": "Vacuolar protein sorting-associated protein 33A",
  "gene_symbol": "VPS33A",
  "gene": "UniProtKB:Q96AX1",
  "term_id": "GO:0033263"
}